{
  "gene_symbol": "PLEKHG7",
  "gene": "UniProtKB:Q6ZR37",
  "term_label": "Unknown biological process",
  "gene_name": "Pleckstrin homology domain-containing family G member 7",
  "term_id": "UNKNOWN:0002"
}